{
  "gene_name": "Zinc finger CCCH domain-containing protein 15",
  "term_label": "cytoplasmic translation",
  "gene": "UniProtKB:Q8WU90",
  "term_id": "GO:0002181",
  "gene_symbol": "ZC3H15"
}